negative regulation of defense response to bacterium [GO:1900425] (biological process) Definition: Any process that stops, prevents or reduces the frequency, rate or extent of defense response to bacterium. References: PMID:22346749 Sources: GOC:TermGenie Also known as: down regulation of defence response to bacteria, down regulation of defence response to bacterium, down regulation of defense response to bacteria, down regulation of defense response to bacterium, down-regulation of defence response to bacteria, down-regulation of defence response to bacterium, down-regulation of defense response to bacteria, down-regulation of defense response to bacterium, downregulation of defence response to bacteria, downregulation of defence response to bacterium, downregulation of defense response to bacteria, downregulation of defense response to bacterium, inhibition of defence response to bacteria, inhibition of defence response to bacterium, inhibition of defense response to bacteria, negative regulation of defence response to bacteria, negative regulation of defence response to bacterium, negative regulation of defense response to bacteria, inhibition of defence response to pathogenic bacteria, incompatible interaction, inhibition of defence response to pathogenic bacterium, incompatible interaction, inhibition of defense response to bacterium, inhibition of defense response to bacterium, incompatible interaction, inhibition of resistance response to pathogenic bacteria, inhibition of resistance response to pathogenic bacterium, inhibition of response to pathogenic bacteria (incompatible interaction), inhibition of response to pathogenic bacterium (incompatible interaction), negative regulation of defense response to bacterium, incompatible interaction, down regulation of antibacterial peptide activity, down-regulation of antibacterial peptide activity, downregulation of antibacterial peptide activity, inhibition of antibacterial peptide activity, negative regulation of antibacterial peptide activity Relationships: is a type of GO:0002832; is a type of GO:0031348; is a type of negative regulation of response to external stimulus [GO:0032102]; is a type of regulation of defense response to bacterium [GO:1900424]; negatively regulates GO:0042742 Subtypes: GO:0002787, negative regulation of peptidoglycan recognition protein signaling pathway [GO:0061060]